{
  "gene_name": "Sperm protein associated with the nucleus on the X chromosome C",
  "term_id": "UNKNOWN:0003",
  "gene": "UniProtKB:Q9NY87",
  "gene_symbol": "SPANXC",
  "term_label": "Unknown cellular component"
}